{
  "term_label": "negative regulation of cell migration involved in sprouting angiogenesis",
  "gene_symbol": "MMRN2",
  "term_id": "GO:0090051",
  "gene_name": "Multimerin-2",
  "gene": "UniProtKB:Q9H8L6"
}